DNA ligase (ATP) activity [GO:0003910] (molecular function) Definition: Catalysis of the reaction: ATP + deoxyribonucleotide(n) + deoxyribonucleotide(m) = AMP + diphosphate + deoxyribonucleotide(n+m). Also known as: DNA joinase activity, deoxyribonucleate ligase, deoxyribonucleic acid joinase, deoxyribonucleic acid ligase, deoxyribonucleic joinase, deoxyribonucleic ligase, polynucleotide ligase, DNA repair enzyme activity, DNA-joining enzyme, deoxyribonucleic acid repair enzyme, deoxyribonucleic acid-joining enzyme, deoxyribonucleic repair enzyme, deoxyribonucleic-joining enzyme, poly(deoxyribonucleotide):poly(deoxyribonucleotide) ligase (AMP-forming), polydeoxyribonucleotide synthase (ATP) activity, polynucleotide ligase (ATP) activity, sealase activity Relationships: is a type of DNA ligase activity [GO:0003909] Sources: EC:6.5.1.1